{
  "gene_symbol": "ATP8A2",
  "term_id": "GO:0048666",
  "term_label": "neuron development",
  "gene": "UniProtKB:Q9NTI2",
  "gene_name": "Phospholipid-transporting ATPase IB"
}